{
  "term_id": "GO:0046875",
  "gene_name": "Ephrin-A3",
  "gene": "UniProtKB:P52797",
  "term_label": "ephrin receptor binding",
  "gene_symbol": "EFNA3"
}